{
  "gene_name": "Mast_stem cell growth factor receptor Kit",
  "gene_symbol": "KIT",
  "term_label": "transmembrane receptor protein tyrosine kinase activity",
  "term_id": "GO:0004714",
  "gene": "UniProtKB:P10721"
}